{
  "gene": "UniProtKB:Q9BU40",
  "gene_name": "Chordin-like protein 1",
  "term_label": "BMP binding",
  "term_id": "GO:0036122",
  "gene_symbol": "CHRDL1"
}